{
  "gene_name": "Annexin A9",
  "gene": "UniProtKB:O76027",
  "term_label": "plasma membrane",
  "term_id": "GO:0005886",
  "gene_symbol": "ANXA9"
}